negative regulation of neutrophil mediated killing of fungus [GO:0070959] (biological process) Sources: GOC:add, GOC:mah Definition: Any process that decreases the frequency, rate or extent of the directed killing of a fungal cell by a neutrophil. Also known as: down regulation of neutrophil mediated killing of fungus, down-regulation of neutrophil mediated killing of fungus, downregulation of neutrophil mediated killing of fungus, inhibition of neutrophil mediated killing of fungus Relationships: is a type of GO:0070953; is a type of GO:0070955; RO_0002212 GO:0070947